regulation of T cell homeostatic proliferation [GO:0046013] (biological process) Sources: GOC:go_curators Also known as: regulation of T lymphocyte homeostatic proliferation, regulation of T-cell homeostatic proliferation, regulation of T-lymphocyte homeostatic proliferation, regulation of resting T cell proliferation Relationships: is a type of GO:0042129; regulates T cell homeostatic proliferation [GO:0001777] Subtypes: positive regulation of T cell homeostatic proliferation [GO:0042103], GO:0046014 Definition: Any process that modulates the frequency, rate or extent of resting T cell proliferation.